{
  "gene_name": "CD320 antigen",
  "gene_symbol": "CD320",
  "gene": "UniProtKB:Q9NPF0",
  "term_id": "UNKNOWN:0001",
  "term_label": "Unknown molecular function"
}